oxaloacetate metabolic process [GO:0006107] (biological process) Definition: The chemical reactions and pathways involving oxaloacetate, the anion of oxobutanedioic acid, an important intermediate in metabolism, especially as a component of the TCA cycle. Also known as: oxaloacetate metabolism Sources: ISBN:0198506732 Relationships: is a type of dicarboxylic acid metabolic process [GO:0043648] Subtypes: L-asparagine biosynthetic process from oxaloacetate [GO:0019266], glutamate catabolic process to oxaloacetate [GO:0019554], protocatechuate catabolic process, meta-cleavage [GO:0019617]